{
  "gene_symbol": "CDC14B",
  "term_id": "GO:0004725",
  "gene_name": "Dual specificity protein phosphatase CDC14B",
  "term_label": "protein tyrosine phosphatase activity",
  "gene": "UniProtKB:O60729"
}